{
  "gene_symbol": "IGLV2-18",
  "term_label": "Unknown molecular function",
  "gene_name": "Immunoglobulin lambda variable 2-18",
  "gene": "UniProtKB:A0A075B6J9",
  "term_id": "UNKNOWN:0001"
}